{
  "gene_symbol": "COX8A",
  "term_id": "GO:0045277",
  "term_label": "respiratory chain complex IV",
  "gene_name": "Cytochrome c oxidase subunit 8A, mitochondrial",
  "gene": "UniProtKB:P10176"
}